{
  "gene_symbol": "LTBP2",
  "gene_name": "Latent-transforming growth factor beta-binding protein 2",
  "gene": "UniProtKB:Q14767",
  "term_id": "GO:0097435",
  "term_label": "supramolecular fiber organization"
}